{
  "gene_name": "Tubulin-folding cofactor B",
  "term_label": "cytoplasmic microtubule organization",
  "gene": "UniProtKB:Q99426",
  "term_id": "GO:0031122",
  "gene_symbol": "TBCB"
}